{
  "gene": "UniProtKB:Q9UKM7",
  "term_id": "GO:0036503",
  "term_label": "ERAD pathway",
  "gene_name": "Endoplasmic reticulum mannosyl-oligosaccharide 1,2-alpha-mannosidase",
  "gene_symbol": "MAN1B1"
}